{
  "term_id": "GO:0001671",
  "gene_symbol": "AHSA2P",
  "term_label": "ATPase activator activity",
  "gene_name": "Putative activator of 90 kDa heat shock protein ATPase homolog 2",
  "gene": "UniProtKB:Q719I0"
}